{
  "gene_name": "Nuclear receptor subfamily 6 group A member 1",
  "term_label": "nuclear receptor activity",
  "gene_symbol": "NR6A1",
  "gene": "UniProtKB:Q15406",
  "term_id": "GO:0004879"
}